{
  "term_id": "UNKNOWN:0001",
  "gene": "UniProtKB:Q16655",
  "gene_symbol": "MLANA",
  "term_label": "Unknown molecular function",
  "gene_name": "Melanoma antigen recognized by T-cells 1"
}